T-helper 2 cell chemotaxis [GO:0035707] (biological process) Definition: The directed movement of a T-helper 2 cell in response to an external stimulus. Relationships: is a type of T cell chemotaxis [GO:0010818] Also known as: Th2 cell chemotaxis Sources: CL:0000546, GOC:BHF